vacuole fission [GO:0140572] (biological process) References: PMID:19643199 Relationships: is a type of GO:0048285 Definition: The division of a vacuole within a cell to form two or more separate vacuoles.